{
  "term_label": "fatty acid biosynthetic process",
  "term_id": "GO:0006633",
  "gene_symbol": "ACSM1",
  "gene": "UniProtKB:Q08AH1",
  "gene_name": "Acyl-coenzyme A synthetase ACSM1, mitochondrial"
}